L-malate dehydrogenase (NAD+) activity [GO:0030060] (molecular function) Relationships: is a type of GO:0016615; is a type of oxidoreductase activity, acting on the CH-OH group of donors, NAD or NADP as acceptor [GO:0016616] Definition: Catalysis of the reaction: (S)-malate + NAD+ = oxaloacetate + NADH + H+. Sources: RHEA:21432 Also known as: NAD-L-malate dehydrogenase activity, (S)-malate:NAD+ oxidoreductase activity, L-malate-NAD+ oxidoreductase activity, MDH, NAD-dependent malate dehydrogenase activity, NAD-dependent malic dehydrogenase activity, NAD-linked malate dehydrogenase activity, NAD-malate dehydrogenase activity, NAD-malic dehydrogenase activity, NAD-specific malate dehydrogenase activity, malate (NAD) dehydrogenase activity, malic acid dehydrogenase activity, malic dehydrogenase activity